{
  "term_id": "GO:0031274",
  "term_label": "positive regulation of pseudopodium assembly",
  "gene_name": "Uncharacterized protein C15orf62, mitochondrial",
  "gene": "UniProtKB:A8K5M9",
  "gene_symbol": "C15orf62"
}